{
  "term_label": "cell-cell adhesion",
  "gene": "UniProtKB:O94856",
  "gene_name": "Neurofascin",
  "gene_symbol": "NFASC",
  "term_id": "GO:0098609"
}